{
  "term_id": "GO:0019780",
  "gene_symbol": "UBA6",
  "gene": "UniProtKB:A0AVT1",
  "gene_name": "Ubiquitin-like modifier-activating enzyme 6",
  "term_label": "FAT10 activating enzyme activity"
}